polarity specification of dorsal/ventral axis [GO:0009951] (biological process) Definition: Any process resulting in the establishment of polarity along the dorsal/ventral axis. Relationships: is a type of specification of axis polarity [GO:0065001]; is part of dorsal/ventral axis specification [GO:0009950] Also known as: polarity specification of dorsal-ventral axis, polarity specification of dorsoventral axis Sources: GOC:go_curators